mismatch repair complex [GO:0032300] (cellular component) Sources: GOC:mah Definition: Any complex formed of proteins that act in mismatch repair. Subtypes: GO:0032301, GO:0032302, GO:0032389, MutLbeta complex [GO:0032390], GO:0062128, GO:0097587, GO:1990710 Relationships: is_a protein-containing complex [GO:0032991]; is part of intracellular anatomical structure [GO:0005622]